{
  "gene": "UniProtKB:Q6P2S7",
  "term_label": "Unknown biological process",
  "gene_symbol": "TTC41P",
  "gene_name": "Putative tetratricopeptide repeat protein 41",
  "term_id": "UNKNOWN:0002"
}